arachidonate 5,6-epoxygenase activity [GO:0106301] (MF) References: PMID:10491410, PMID:8631948 Sources: RHEA:49936 Relationships: is a type of arachidonate epoxygenase activity [GO:0008392] Also known as: arachidonic acid 5,6-epoxygenase activity Definition: Catalysis of an NADPH- and oxygen-dependent reaction that converts arachidonic acid to cis-5,6-epoxyeicosatrienoic acid.